monoatomic anion:sodium symporter activity [GO:0015373] (molecular function) Also known as: anion:sodium symporter activity, monovalent anion:sodium symporter activity Definition: Enables the transfer of a solute or solutes from one side of a membrane to the other according to the reaction: monoatomic anion(out) + Na+(out) = monoatomic anion(in) + Na+(in). Subtypes: sodium:iodide symporter activity [GO:0008507], GO:0015378 Sources: TC:2.A.21.5.- Relationships: is_a monoatomic anion:monoatomic cation symporter activity [GO:0015296]; is_a solute:sodium symporter activity [GO:0015370]